multicellular organismal-level homeostasis [GO:0048871] (biological process) Definition: Any process involved in the maintenance of an internal steady state at the level of the multicellular organism. Sources: GOC:isa_complete Relationships: is a type of multicellular organismal process [GO:0032501]; is a type of homeostatic process [GO:0042592] Subtypes: temperature homeostasis [GO:0001659], GO:0048872, anatomical structure homeostasis [GO:0060249], energy homeostasis [GO:0097009], GO:0140962, GO:0160060, respiratory chemosensitivity [GO:0160061]